{
  "gene_name": "La-related protein 7",
  "term_id": "UNKNOWN:0003",
  "gene_symbol": "LARP7",
  "term_label": "Unknown cellular component",
  "gene": "UniProtKB:Q4G0J3"
}